{
  "term_id": "GO:0036064",
  "gene_symbol": "CEP19",
  "term_label": "ciliary basal body",
  "gene": "UniProtKB:Q96LK0",
  "gene_name": "Centrosomal protein of 19 kDa"
}